{
  "gene": "UniProtKB:O15427",
  "term_id": "UNKNOWN:0002",
  "term_label": "Unknown biological process",
  "gene_symbol": "SLC16A3",
  "gene_name": "Monocarboxylate transporter 4"
}